negative regulation of endothelial cell apoptotic process [GO:2000352] (biological process) Sources: GOC:BHF, GOC:mah, GOC:mtg_apoptosis Relationships: is a type of negative regulation of apoptotic process [GO:0043066]; is a type of regulation of endothelial cell apoptotic process [GO:2000351]; negatively regulates endothelial cell apoptotic process [GO:0072577] Also known as: negative regulation of apoptosis of endothelial cells, negative regulation of endothelial cell programmed cell death by apoptosis, negative regulation of killing of endothelial cells, negative regulation of programmed cell death of endothelial cells by apoptosis, negative regulation of programmed cell death, endothelial cells, negative regulation of endothelial cell apoptosis Definition: Any process that stops, prevents or reduces the frequency, rate or extent of endothelial cell apoptotic process.